{
  "gene_symbol": "KRTAP19-4",
  "term_label": "Unknown biological process",
  "gene_name": "Keratin-associated protein 19-4",
  "gene": "UniProtKB:Q3LI73",
  "term_id": "UNKNOWN:0002"
}